spongiotrophoblast layer development [GO:0060712] (biological process) Definition: The process in which the spongiotrophoblast layer of the placenta progresses from its formation to its mature state. Sources: GOC:dph Relationships: is a type of tissue development [GO:0009888]; is part of embryonic placenta development [GO:0001892]